{
  "gene_name": "Integrin beta-2",
  "term_label": "cell surface",
  "term_id": "GO:0009986",
  "gene": "UniProtKB:P05107",
  "gene_symbol": "ITGB2"
}